{
  "term_id": "GO:0030198",
  "gene_symbol": "MMP21",
  "term_label": "extracellular matrix organization",
  "gene": "UniProtKB:Q8N119",
  "gene_name": "Matrix metalloproteinase-21"
}